{
  "gene_symbol": "TPT1P8",
  "gene_name": "Putative translationally-controlled tumor protein-like protein TPT1P8",
  "gene": "UniProtKB:Q9HAU6",
  "term_label": "calcium ion binding",
  "term_id": "GO:0005509"
}